negative regulation of telomere maintenance [GO:0032205] (biological process) Definition: Any process that stops, prevents, or reduces the frequency, rate or extent of a process that affects and monitors the activity of telomeric proteins and the length of telomeric DNA. Also known as: down regulation of telomere maintenance, down-regulation of telomere maintenance, downregulation of telomere maintenance, inhibition of telomere maintenance Relationships: is a type of regulation of telomere maintenance [GO:0032204]; is a type of negative regulation of DNA metabolic process [GO:0051053]; is a type of GO:2001251; negatively regulates telomere maintenance [GO:0000723] Sources: GOC:mah Subtypes: GO:0032208, negative regulation of telomere maintenance via semi-conservative replication [GO:0032214], negative regulation of telomere capping [GO:1904354], negative regulation of telomere maintenance via telomere lengthening [GO:1904357], negative regulation of telomeric loop formation [GO:1904419], negative regulation of telomere maintenance in response to DNA damage [GO:1904506], negative regulation of telomeric loop disassembly [GO:1904534]